{
  "gene_name": "ATP-dependent 6-phosphofructokinase, muscle type",
  "term_label": "fructose 6-phosphate metabolic process",
  "gene": "UniProtKB:P08237",
  "term_id": "GO:0006002",
  "gene_symbol": "PFKM"
}